N',N'',N'''-triacetylfusarinine C catabolic process [GO:1900550] (biological process) Relationships: is a type of secondary metabolite catabolic process [GO:0090487] Also known as: N',N'',N'''-triacetylfusarinine C breakdown, N',N'',N'''-triacetylfusarinine C catabolism, N',N'',N'''-triacetylfusarinine C degradation Definition: The chemical reactions and pathways resulting in the breakdown of N',N'',N'''-triacetylfusarinine C. Sources: GOC:TermGenie, GOC:di